{
  "gene_name": "Proprotein convertase subtilisin_kexin type 5",
  "gene": "UniProtKB:Q92824",
  "gene_symbol": "PCSK5",
  "term_label": "trans-Golgi network",
  "term_id": "GO:0005802"
}